asexual sporulation resulting in formation of a multicellular or syncytial spore [GO:0075284] (biological process) Relationships: is a type of GO:0030436; is a type of sporulation resulting in formation of a multicellular or syncytial spore [GO:0075283] Definition: The formation of a multicellular or syncytial spore via septations derived from mitosis. Sources: GOC:pamgo_curators